{
  "gene": "UniProtKB:A0A1B0GUQ0",
  "term_id": "UNKNOWN:0001",
  "gene_name": "Protein FAM236A",
  "gene_symbol": "FAM236A",
  "term_label": "Unknown molecular function"
}